{
  "gene": "UniProtKB:Q66K79",
  "term_id": "GO:0006518",
  "gene_symbol": "CPZ",
  "gene_name": "Carboxypeptidase Z",
  "term_label": "peptide metabolic process"
}